{
  "gene_symbol": "ZNF92",
  "term_id": "GO:0000978",
  "gene": "UniProtKB:Q03936",
  "gene_name": "Zinc finger protein 92",
  "term_label": "RNA polymerase II cis-regulatory region sequence-specific DNA binding"
}